{
  "term_id": "GO:0005794",
  "gene_symbol": "TMED10",
  "gene_name": "Transmembrane emp24 domain-containing protein 10",
  "term_label": "Golgi apparatus",
  "gene": "UniProtKB:P49755"
}